{
  "gene_name": "Serine_threonine-protein kinase ULK1",
  "term_label": "axon extension",
  "gene_symbol": "ULK1",
  "gene": "UniProtKB:O75385",
  "term_id": "GO:0048675"
}